violaceol I metabolic process [GO:1900588] (biological process) Definition: The chemical reactions and pathways involving violaceol I. Also known as: violaceol I metabolism Relationships: is a type of catechol-containing compound metabolic process [GO:0009712]; is a type of secondary metabolic process [GO:0019748] Subtypes: violaceol I catabolic process [GO:1900589], violaceol I biosynthetic process [GO:1900590] Sources: GOC:TermGenie, GOC:di